negative regulation of Kit signaling pathway [GO:1900235] (biological process) Also known as: down regulation of Kit signaling pathway, down regulation of stem cell factor receptor signaling pathway, down regulation of stem cell factor signaling pathway, down-regulation of Kit signaling pathway, down-regulation of stem cell factor receptor signaling pathway, down-regulation of stem cell factor signaling pathway, downregulation of Kit signaling pathway, downregulation of stem cell factor receptor signaling pathway, downregulation of stem cell factor signaling pathway, inhibition of stem cell factor receptor signaling pathway, inhibition of stem cell factor signaling pathway, negative regulation of Kit signalling pathway, negative regulation of stem cell factor receptor signaling pathway, negative regulation of stem cell factor signaling pathway, inhibition of Kit signaling pathway Sources: GOC:TermGenie, GOC:signaling Definition: Any process that stops, prevents or reduces the frequency, rate or extent of Kit signaling pathway. Relationships: is a type of negative regulation of cytokine-mediated signaling pathway [GO:0001960]; is_a regulation of Kit signaling pathway [GO:1900234]; negatively regulates GO:0038109